{
  "gene": "UniProtKB:P61006",
  "term_id": "GO:0030140",
  "gene_symbol": "RAB8A",
  "gene_name": "Ras-related protein Rab-8A",
  "term_label": "trans-Golgi network transport vesicle"
}